thyroid-stimulating hormone receptor activity [GO:0004996] (molecular function) Definition: Combining with thyroid-stimulating hormone to initiate a change in cell activity. Sources: GOC:mah Relationships: is a type of GO:0004930; is a type of GO:0016500; is part of thyroid-stimulating hormone signaling pathway [GO:0038194] Also known as: TSH receptor activity, thyroid stimulating hormone receptor activity, thyrotropin receptor